cytoplasmic side of lysosomal membrane [GO:0098574] (CC) Also known as: external leaflet of lysosomal membrane, external side of lysosomal membrane Sources: GOC:ab, GOC:dos Relationships: is a type of GO:0098562; is part of lysosomal membrane [GO:0005765] Definition: The side (leaflet) of the lysosomal membrane that faces the cytoplasm.